{
  "gene_name": "UDP-N-acetylglucosamine transferase subunit ALG14 homolog",
  "term_id": "GO:0006488",
  "gene": "UniProtKB:Q96F25",
  "term_label": "dolichol-linked oligosaccharide biosynthetic process",
  "gene_symbol": "ALG14"
}